{
  "gene_symbol": "CYB5R3",
  "gene": "UniProtKB:P00387",
  "term_label": "cytochrome-b5 reductase activity, acting on NAD(P)H",
  "term_id": "GO:0004128",
  "gene_name": "NADH-cytochrome b5 reductase 3"
}